{
  "term_label": "dendrite",
  "gene_name": "Ephrin type-A receptor 8",
  "gene_symbol": "EPHA8",
  "term_id": "GO:0030425",
  "gene": "UniProtKB:P29322"
}